{
  "gene_name": "Pleckstrin homology domain-containing family A member 4",
  "gene": "UniProtKB:Q9H4M7",
  "term_id": "GO:0005546",
  "gene_symbol": "PLEKHA4",
  "term_label": "phosphatidylinositol-4,5-bisphosphate binding"
}